{
  "gene_symbol": "CAD",
  "term_id": "GO:0004088",
  "gene_name": "CAD protein",
  "gene": "UniProtKB:P27708",
  "term_label": "carbamoyl-phosphate synthase (glutamine-hydrolyzing) activity"
}